{
  "gene": "UniProtKB:Q01955",
  "term_label": "extracellular matrix organization",
  "gene_name": "Collagen alpha-3(IV) chain",
  "term_id": "GO:0030198",
  "gene_symbol": "COL4A3"
}